{
  "gene": "UniProtKB:P06576",
  "term_id": "GO:0042776",
  "gene_symbol": "ATP5F1B",
  "gene_name": "ATP synthase subunit beta, mitochondrial",
  "term_label": "proton motive force-driven mitochondrial ATP synthesis"
}